{
  "gene": "UniProtKB:O60242",
  "gene_symbol": "ADGRB3",
  "gene_name": "Adhesion G protein-coupled receptor B3",
  "term_label": "G protein-coupled receptor signaling pathway",
  "term_id": "GO:0007186"
}